neuronal pentraxin receptor activity [GO:0008030] (MF) Definition: Combining with a neuronal pentraxin and transmitting the signal from one side of the membrane to the other to initiate a change in cell activity. References: PMID:18840757 Sources: GOC:mah, GOC:signaling Relationships: is a type of pentraxin receptor activity [GO:0008029] Also known as: neuronal pentaxin receptor